{
  "gene": "UniProtKB:Q9NRP7",
  "term_id": "GO:0005737",
  "gene_symbol": "STK36",
  "gene_name": "Serine_threonine-protein kinase 36",
  "term_label": "cytoplasm"
}